tooth placode formation [GO:0060790] (biological process) Sources: GOC:dph, GOC:sdb_2009, GOC:tb Relationships: is a type of ectodermal placode formation [GO:0060788]; BFO_0000050 odontogenesis of dentin-containing tooth [GO:0042475] Definition: The developmental process in which the tooth placode forms. A tooth placode is a thickening of the ectoderm that will give rise to the tooth bud.